{
  "gene_name": "ERI1 exoribonuclease 2",
  "gene_symbol": "ERI2",
  "term_label": "Unknown cellular component",
  "term_id": "UNKNOWN:0003",
  "gene": "UniProtKB:A8K979"
}